{
  "gene": "UniProtKB:Q9Y614",
  "term_id": "GO:0005634",
  "term_label": "nucleus",
  "gene_name": "Actin-like protein 7B",
  "gene_symbol": "ACTL7B"
}